{
  "gene_symbol": "AEBP1",
  "term_id": "UNKNOWN:0003",
  "term_label": "Unknown cellular component",
  "gene_name": "Adipocyte enhancer-binding protein 1",
  "gene": "UniProtKB:Q8IUX7"
}